{
  "gene_symbol": "HAS1",
  "term_label": "hyaluronan synthase activity",
  "gene_name": "Hyaluronan synthase 1",
  "term_id": "GO:0050501",
  "gene": "UniProtKB:Q92839"
}